cerebral cortex radial glia-guided migration [GO:0021801] (biological process) Relationships: is a type of GO:0021799; is a type of telencephalon glial cell migration [GO:0022030] Definition: The radial migration of neuronal or glial precursor cells along radial glial cells during the development of the cerebral cortex. Subtypes: pyramidal neuron migration to cerebral cortex [GO:0021852] Also known as: cerebral cortex radial glia guided migration, cerebral cortex radial glia-dependent cell migration, glial-guided locomotion References: PMID:12626695 Sources: GOC:cls, GOC:dgh, GOC:dph, GOC:jid, GO_REF:0000021